phosphoethanolamine phosphatase activity [GO:0052732] (molecular function) Definition: Catalysis of the reaction: phosphoethanolamine + H2O = ethanolamine + phosphate. Sources: RHEA:16089 Also known as: 3X11A, PHOSPHO1, phosphoethanolamine phosphohydrolase activity Relationships: is a type of phosphatase activity [GO:0016791]